{
  "gene_name": "Leucine-rich repeat-containing protein 46",
  "gene": "UniProtKB:Q96FV0",
  "term_id": "UNKNOWN:0003",
  "gene_symbol": "LRRC46",
  "term_label": "Unknown cellular component"
}